{
  "term_id": "GO:0005737",
  "gene_name": "Tyrosine-protein phosphatase non-receptor type 11",
  "gene": "UniProtKB:Q06124",
  "term_label": "cytoplasm",
  "gene_symbol": "PTPN11"
}